{
  "gene": "UniProtKB:Q96AC6",
  "gene_symbol": "KIFC2",
  "term_label": "microtubule binding",
  "gene_name": "Kinesin-like protein KIFC2",
  "term_id": "GO:0008017"
}